methane biosynthetic process from trimethylamine [GO:2001130] (biological process) Definition: The chemical reactions and pathways resulting in the formation of a methane from a trimethylamine. Sources: GOC:mengo_curators Relationships: is a type of GO:0009308; is a type of methanogenesis [GO:0015948] Regulation: regulated by regulation of methane biosynthetic process from trimethylamine [GO:1900330]; negatively regulated by negative regulation of methane biosynthetic process from trimethylamine [GO:1900331]; positively regulated by GO:1900332